{
  "gene": "UniProtKB:Q06323",
  "term_id": "GO:0061133",
  "gene_symbol": "PSME1",
  "term_label": "endopeptidase activator activity",
  "gene_name": "Proteasome activator complex subunit 1"
}